{
  "gene": "UniProtKB:P08922",
  "gene_symbol": "ROS1",
  "gene_name": "Proto-oncogene tyrosine-protein kinase ROS",
  "term_id": "GO:0005886",
  "term_label": "plasma membrane"
}